macromolecule localization [GO:0033036] (biological process) Sources: GOC:mah Relationships: is a type of GO:0051179 Subtypes: RNA localization [GO:0006403], intracellular protein localization [GO:0008104], GO:0010876, protein-containing complex localization [GO:0031503], polysaccharide localization [GO:0033037], lipoprotein localization [GO:0044872], GO:0052575, GO:0071692 Definition: Any process in which a macromolecule is transported to, or maintained in, a specific location. Also known as: macromolecule localisation